hydrogenosome lumen [GO:0034492] (cellular component) Relationships: is a type of intracellular organelle lumen [GO:0070013]; BFO_0000050 hydrogenosome [GO:0042566] Definition: The volume enclosed by the hydrogenosome membrane. Sources: GOC:rph